regulation of spontaneous synaptic transmission [GO:0150003] (biological process) Relationships: is a type of modulation of chemical synaptic transmission [GO:0050804]; regulates GO:0098814 Definition: Any process that modulates the frequency, rate or extent of spontaneous synaptic transmission. Subtypes: GO:1904048 References: PMID:15457210 Sources: GOC:aruk, GOC:bc